{
  "term_id": "GO:0047874",
  "term_label": "dolichyldiphosphatase activity",
  "gene_symbol": "DOLPP1",
  "gene": "UniProtKB:Q86YN1",
  "gene_name": "Dolichyldiphosphatase 1"
}